{
  "gene": "UniProtKB:P33241",
  "gene_name": "Lymphocyte-specific protein 1",
  "term_id": "UNKNOWN:0002",
  "gene_symbol": "LSP1",
  "term_label": "Unknown biological process"
}